maltose epimerase activity [GO:0050558] (molecular function) Definition: Catalysis of the reaction: alpha-maltose = beta-maltose. Relationships: is a type of racemase and epimerase activity, acting on carbohydrates and derivatives [GO:0016857] Sources: EC:5.1.3.21, RHEA:21228 Also known as: maltose 1-epimerase activity